{
  "term_label": "dolichyl-phosphate-mannose-protein mannosyltransferase activity",
  "gene_name": "Protein O-mannosyl-transferase 2",
  "gene_symbol": "POMT2",
  "term_id": "GO:0004169",
  "gene": "UniProtKB:Q9UKY4"
}